{
  "gene_symbol": "C0HLV8",
  "term_label": "Unknown biological process",
  "term_id": "UNKNOWN:0002",
  "gene_name": "PTEN upstream open reading frame MP31",
  "gene": "UniProtKB:C0HLV8"
}